{
  "term_id": "GO:0070098",
  "term_label": "chemokine-mediated signaling pathway",
  "gene": "UniProtKB:Q07325",
  "gene_symbol": "CXCL9",
  "gene_name": "C-X-C motif chemokine 9"
}